{
  "term_id": "GO:0005737",
  "gene_name": "Caspase-6",
  "gene_symbol": "CASP6",
  "term_label": "cytoplasm",
  "gene": "UniProtKB:P55212"
}